{
  "gene": "UniProtKB:Q8TBR4",
  "term_id": "UNKNOWN:0003",
  "gene_name": "Putative STAG3-like protein 4",
  "gene_symbol": "STAG3L4",
  "term_label": "Unknown cellular component"
}